{
  "term_id": "GO:0000122",
  "gene": "UniProtKB:Q14192",
  "gene_name": "Four and a half LIM domains protein 2",
  "term_label": "negative regulation of transcription by RNA polymerase II",
  "gene_symbol": "FHL2"
}